{
  "gene": "UniProtKB:Q9P2G4",
  "gene_name": "Microtubule-associated protein 10",
  "term_id": "GO:0032467",
  "gene_symbol": "MAP10",
  "term_label": "positive regulation of cytokinesis"
}